RNA polymerase III preinitiation complex assembly [GO:0070898] (biological process) Also known as: RNA polymerase III transcription PIC biosynthesis, RNA polymerase III transcription PIC formation, RNA polymerase III transcriptional preinitiation complex assembly, RNA polymerase III transcriptional preinitiation complex formation, RNA polymerase III hybrid type promoter transcriptional preinitiation complex assembly, RNA polymerase III type 1 promoter transcriptional preinitiation complex assembly, RNA polymerase III type 2 promoter transcriptional preinitiation complex assembly, RNA polymerase III type 3 promoter transcriptional preinitiation complex assembly References: PMID:11387215, PMID:12381659 Sources: GOC:txnOH Definition: The formation of a large multiprotein-DNA complex that self-assembles on a tRNA gene through the sequential recruitment of the general initiation factors that compose the preinitiation complex (PIC), (which includes BDP1, BRF1, TBP, TFIIIC in human). The PIC engages RNA polymerase III on its DNA template strand and sparks polymerization of the first few RNA nucleotides. Relationships: is a type of transcription preinitiation complex assembly [GO:0070897]; is part of transcription initiation at RNA polymerase III promoter [GO:0006384]